{
  "gene_symbol": "CNOT7",
  "term_label": "P-body",
  "gene": "UniProtKB:Q9UIV1",
  "gene_name": "CCR4-NOT transcription complex subunit 7",
  "term_id": "GO:0000932"
}